{
  "gene_name": "Unconventional myosin-XIX",
  "gene": "UniProtKB:Q96H55",
  "term_label": "membrane",
  "gene_symbol": "MYO19",
  "term_id": "GO:0016020"
}